macromolecule deacylation [GO:0098732] (biological process) Definition: The removal of an acyl group, any group or radical of the form RCO- where R is an organic group, from a macromolecule. Sources: GOC:dos Relationships: is a type of macromolecule modification [GO:0043412] Subtypes: protein deacylation [GO:0035601], GO:0098734, polyamine deacetylation [GO:0106047]